{
  "gene_name": "Gastrin_cholecystokinin type B receptor",
  "term_id": "GO:0004951",
  "gene_symbol": "CCKBR",
  "term_label": "cholecystokinin receptor activity",
  "gene": "UniProtKB:P32239"
}